{
  "gene_symbol": "PIGY",
  "gene": "UniProtKB:Q3MUY2",
  "gene_name": "Phosphatidylinositol N-acetylglucosaminyltransferase subunit Y",
  "term_label": "Unknown molecular function",
  "term_id": "UNKNOWN:0001"
}